{
  "gene_symbol": "TRIM68",
  "gene": "UniProtKB:Q6AZZ1",
  "term_label": "cytosol",
  "gene_name": "E3 ubiquitin-protein ligase TRIM68",
  "term_id": "GO:0005829"
}